{
  "gene_symbol": "SMIM15",
  "term_label": "Unknown molecular function",
  "gene_name": "Small integral membrane protein 15",
  "gene": "UniProtKB:Q7Z3B0",
  "term_id": "UNKNOWN:0001"
}